{
  "term_id": "GO:0061630",
  "term_label": "ubiquitin protein ligase activity",
  "gene_name": "E3 ubiquitin-protein ligase TRIM68",
  "gene_symbol": "TRIM68",
  "gene": "UniProtKB:Q6AZZ1"
}